{
  "gene_name": "Interferon alpha-16",
  "gene": "UniProtKB:P05015",
  "gene_symbol": "IFNA16",
  "term_id": "GO:0006959",
  "term_label": "humoral immune response"
}